{
  "gene_symbol": "IL3",
  "term_label": "extracellular space",
  "term_id": "GO:0005615",
  "gene": "UniProtKB:P08700",
  "gene_name": "Interleukin-3"
}